{
  "gene_symbol": "ANO6",
  "term_label": "chloride transmembrane transport",
  "gene": "UniProtKB:Q4KMQ2",
  "gene_name": "Anoctamin-6",
  "term_id": "GO:1902476"
}